{
  "gene_name": "Thy-1 membrane glycoprotein",
  "term_label": "dendrite",
  "gene_symbol": "THY1",
  "term_id": "GO:0030425",
  "gene": "UniProtKB:P04216"
}